{
  "gene_symbol": "DDR2",
  "gene_name": "Discoidin domain-containing receptor 2",
  "term_id": "GO:0038062",
  "term_label": "protein tyrosine kinase collagen receptor activity",
  "gene": "UniProtKB:Q16832"
}